G1 phase [GO:0051318] (biological process) Note: Note that this term should not be used for direct annotation. If you are trying to make an annotation to x phase, it is likely that the correct annotation is 'regulation of x/y phase transition' or to a process which occurs during the reported phase (i.e mitotic DNA replication for mitotic S-phase). To capture the phase when a specific location or process is observed, the phase term can be used in an annotation extension (PMID:24885854) applied to a cellular component term (with the relation exists_during) or a biological process term (with the relation happens_during). Sources: GOC:mtg_cell_cycle Relationships: is a type of GO:0022403; is part of interphase [GO:0051325] Definition: The cell cycle 'gap' phase which is the interval between the completion of DNA segregation (usually by mitosis or meiosis) and the beginning of DNA synthesis. Subtypes: mitotic G1 phase [GO:0000080], meiotic G1 phase [GO:0051330]